regulation of digestive system process [GO:0044058] (BP) Definition: Any process that modulates the frequency, rate or extent of a digestive system process, a physical, chemical, or biochemical process carried out by living organisms to break down ingested nutrients into components that may be easily absorbed and directed into metabolism. Subtypes: regulation of hindgut contraction [GO:0043134], regulation of saliva secretion [GO:0046877], regulation of gastric acid secretion [GO:0060453], positive regulation of digestive system process [GO:0060456], negative regulation of digestive system process [GO:0060457], regulation of intestinal epithelial structure maintenance [GO:0060730], regulation of pancreatic juice secretion [GO:0090186], regulation of small intestinal transit [GO:0120057], regulation of intestinal absorption [GO:1904478], regulation of gastric motility [GO:1905333], regulation of defecation [GO:2000292] Relationships: is a type of regulation of system process [GO:0044057]; RO_0002211 digestive system process [GO:0022600] Sources: GOC:jl